negative regulation of protein insertion into mitochondrial outer membrane [GO:1903637] (biological process) References: PMID:16374546 Sources: GOC:TermGenie, GO_REF:0000058 Relationships: is a type of negative regulation of organelle organization [GO:0010639]; is a type of GO:1903215; is a type of GO:1903636; negatively regulates protein insertion into mitochondrial outer membrane [GO:0045040] Definition: Any process that stops, prevents or reduces the frequency, rate or extent of protein insertion into mitochondrial outer membrane. Also known as: down regulation of mitochondrial outer membrane protein import, down regulation of protein import into mitochondrial outer membrane, down regulation of protein insertion into mitochondrial outer membrane, down regulation of protein transport into mitochondrial outer membrane, down-regulation of mitochondrial outer membrane protein import, down-regulation of protein import into mitochondrial outer membrane, down-regulation of protein insertion into mitochondrial outer membrane, down-regulation of protein transport into mitochondrial outer membrane, downregulation of mitochondrial outer membrane protein import, downregulation of protein import into mitochondrial outer membrane, downregulation of protein insertion into mitochondrial outer membrane, downregulation of protein transport into mitochondrial outer membrane, negative regulation of mitochondrial outer membrane protein import, negative regulation of protein import into mitochondrial outer membrane, negative regulation of protein transport into mitochondrial outer membrane, inhibition of mitochondrial outer membrane protein import, inhibition of protein import into mitochondrial outer membrane, inhibition of protein insertion into mitochondrial outer membrane, inhibition of protein transport into mitochondrial outer membrane